{
  "gene": "UniProtKB:F8WFD2",
  "gene_name": "Nuclear pore complex-interacting protein family member A3",
  "term_id": "UNKNOWN:0001",
  "gene_symbol": "NPIPA3",
  "term_label": "Unknown molecular function"
}